{
  "gene": "UniProtKB:Q9NZ63",
  "gene_symbol": "C9orf78",
  "gene_name": "Splicing factor C9orf78",
  "term_label": "mRNA splicing, via spliceosome",
  "term_id": "GO:0000398"
}